{
  "gene_symbol": "ARHGDIB",
  "term_label": "Rho GDP-dissociation inhibitor activity",
  "gene_name": "Rho GDP-dissociation inhibitor 2",
  "term_id": "GO:0005094",
  "gene": "UniProtKB:P52566"
}